{
  "gene_symbol": "CRKL",
  "gene": "UniProtKB:P46109",
  "term_id": "GO:0007167",
  "term_label": "enzyme-linked receptor protein signaling pathway",
  "gene_name": "Crk-like protein"
}